{
  "term_label": "sodium channel regulator activity",
  "term_id": "GO:0017080",
  "gene_name": "Sodium_potassium-transporting ATPase subunit gamma",
  "gene_symbol": "FXYD2",
  "gene": "UniProtKB:P54710"
}